{
  "gene_name": "Interleukin-1 receptor accessory protein-like 1",
  "gene_symbol": "IL1RAPL1",
  "term_label": "cell surface",
  "term_id": "GO:0009986",
  "gene": "UniProtKB:Q9NZN1"
}